{
  "term_label": "Unknown cellular component",
  "gene_symbol": "SLFN13",
  "gene": "UniProtKB:Q68D06",
  "gene_name": "Schlafen family member 13",
  "term_id": "UNKNOWN:0003"
}